{
  "gene_symbol": "TBC1D3H",
  "term_id": "UNKNOWN:0002",
  "term_label": "Unknown biological process",
  "gene": "UniProtKB:P0C7X1",
  "gene_name": "TBC1 domain family member 3H"
}